cellular response to interleukin-18 [GO:0071351] (biological process) Sources: GOC:mah Also known as: cellular response to IL-18 Relationships: is a type of GO:0070673; is a type of GO:0071345 Definition: Any process that results in a change in state or activity of a cell (in terms of movement, secretion, enzyme production, gene expression, etc.) as a result of an interleukin-18 stimulus.